{
  "gene_name": "Molybdenum cofactor biosynthesis protein 1",
  "gene": "UniProtKB:Q9NZB8",
  "term_label": "Unknown cellular component",
  "term_id": "UNKNOWN:0003",
  "gene_symbol": "MOCS1"
}